{
  "term_label": "serine-type endopeptidase activity",
  "gene_name": "Haptoglobin",
  "gene_symbol": "HP",
  "term_id": "GO:0004252",
  "gene": "UniProtKB:P00738"
}